iron-responsive element binding [GO:0030350] (molecular function) References: PMID:3198610, PMID:8710843 Definition: Binding to an iron-responsive element, a regulatory sequence found in the 5'- and 3'-untranslated regions of mRNAs encoding many iron-binding proteins. Relationships: is a type of mRNA binding [GO:0003729] Also known as: IRE binding